{
  "term_id": "GO:0005549",
  "term_label": "odorant binding",
  "gene_symbol": "OR10W1",
  "gene": "UniProtKB:Q8NGF6",
  "gene_name": "Olfactory receptor 10W1"
}